{
  "gene_symbol": "TSBP1",
  "term_id": "UNKNOWN:0003",
  "term_label": "Unknown cellular component",
  "gene": "UniProtKB:Q5SRN2",
  "gene_name": "Testis-expressed basic protein 1"
}